{
  "term_id": "GO:0071051",
  "gene_symbol": "EXOSC4",
  "gene": "UniProtKB:Q9NPD3",
  "term_label": "poly(A)-dependent snoRNA 3'-end processing",
  "gene_name": "Exosome complex component RRP41"
}